{
  "gene_name": "Lon protease homolog, mitochondrial",
  "gene": "UniProtKB:P36776",
  "term_label": "protein quality control for misfolded or incompletely synthesized proteins",
  "gene_symbol": "LONP1",
  "term_id": "GO:0006515"
}